{
  "gene_symbol": "CLTC",
  "gene": "UniProtKB:Q00610",
  "term_label": "clathrin coat assembly",
  "term_id": "GO:0048268",
  "gene_name": "Clathrin heavy chain 1"
}